outflow tract septum morphogenesis [GO:0003148] (biological process) Relationships: is a type of cardiac septum morphogenesis [GO:0060411]; is part of GO:0003151 Definition: The process in which the anatomical structures of the outflow tract septum are generated and organized. The outflow tract septum is a partition in the outflow tract. Sources: GOC:mtg_heart